FBXO family protein binding [GO:0098770] (molecular function) References: PMID:11178263 Relationships: is a type of protein binding [GO:0005515] Definition: Binding to a member of the FBXO protein family. Members of this family have an F-box protein motif of approximately 50 amino acids that functions as a site of protein-protein interaction.